regulation of L-proline biosynthetic process [GO:1902005] (biological process) Subtypes: GO:1902006 Relationships: is a type of regulation of L-proline metabolic process [GO:2000214]; is a type of regulation of amino acid biosynthetic process [GO:2000282]; regulates GO:0055129 Definition: Any process that modulates the frequency, rate or extent of L-proline biosynthetic process. Also known as: regulation of proline biosynthetic process, regulation of proline anabolism, regulation of proline biosynthesis, regulation of proline formation, regulation of proline synthesis References: PMID:23415322 Sources: GOC:TermGenie